{
  "gene_symbol": "GBP7",
  "term_label": "GTP binding",
  "gene_name": "Guanylate-binding protein 7",
  "term_id": "GO:0005525",
  "gene": "UniProtKB:Q8N8V2"
}